{
  "gene": "UniProtKB:Q9HCM2",
  "term_id": "GO:0002116",
  "term_label": "semaphorin receptor complex",
  "gene_name": "Plexin-A4",
  "gene_symbol": "PLXNA4"
}